socially cooperative development [GO:0099120] (biological process) Relationships: is a type of anatomical structure development [GO:0048856]; is a type of biological process involved in intraspecies interaction between organisms [GO:0051703] Also known as: colonial development, socially co-operative development, non-reproductive fruiting body development References: PMID:12448714 Sources: GOC:pf Definition: The process whose specific outcome is the progression of a non-reproductive fruiting body over time, from its formation to the mature structure. A non-reproductive fruiting body is a colonial multicellular structure consisting of co-operating unicellular organisms, some of which are spores. An example of such a process is found in Dictyostelium discoideum and Myxococcus xanthus colonies. Subtypes: sorocarp development [GO:0030587], GO:0031150, aggregation involved in sorocarp development [GO:0031152], GO:0031153, culmination involved in sorocarp development [GO:0031154], sorocarp sorus development [GO:0048837], chimeric colonial development [GO:0099135]